{
  "gene_name": "HLA class I histocompatibility antigen, B alpha chain",
  "term_label": "positive regulation of T cell mediated cytotoxicity",
  "gene": "UniProtKB:P01889",
  "term_id": "GO:0001916",
  "gene_symbol": "HLA-B"
}